protein-glutamine N-methyltransferase activity [GO:0036009] (molecular function) Also known as: protein glutamine N-methylase activity, protein glutamine N-methyltransferase activity Subtypes: peptide chain release factor N(5)-glutamine methyltransferase activity [GO:0102559], GO:1990259 References: PMID:11847124 Sources: RHEA:57452 Relationships: is_a N-methyltransferase activity [GO:0008170]; is_a GO:0008276; is a type of S-adenosylmethionine-dependent methyltransferase activity [GO:0008757] Definition: Catalysis of the reaction: L-glutaminyl-[protein] + S-adenosyl-L-methionine = N(5)-methyl-L-glutaminyl-[protein] + S-adenosyl-L-homocysteine + H+.